GDP-L-fucose salvage [GO:0042352] (biological process) Sources: GOC:ma Definition: The formation of GDP-L-fucose from L-fucose, without de novo synthesis. L-fucose is phosphorylated by fucokinase and then converted by fucose-1-phosphate guanylyltransferase (EC:2.7.7.30). Also known as: GDP-L-fucose biosynthesis, salvage pathway, GDP-L-fucose biosynthetic process, salvage pathway Relationships: is a type of GO:0042350; is a type of metabolic compound salvage [GO:0043094]